{
  "term_label": "Unknown molecular function",
  "gene": "UniProtKB:Q5VTL7",
  "gene_name": "Fibronectin type III domain-containing protein 7",
  "gene_symbol": "FNDC7",
  "term_id": "UNKNOWN:0001"
}